arylformamidase activity [GO:0004061] (molecular function) Definition: Catalysis of the reaction: N-formyl-L-kynurenine + H2O = formate + L-kynurenine. Relationships: is_a hydrolase activity, acting on carbon-nitrogen (but not peptide) bonds, in linear amides [GO:0016811] Sources: EC:3.5.1.9 Also known as: aryl-formylamine amidohydrolase activity, formamidase I, formamidase II, formylase activity, formylkynureninase activity, formylkynurenine formamidase activity, kynurenine formamidase activity